{
  "term_id": "GO:0099560",
  "gene": "UniProtKB:Q9ULB4",
  "gene_name": "Cadherin-9",
  "term_label": "synaptic membrane adhesion",
  "gene_symbol": "CDH9"
}